minus-end-directed microtubule motor activity [GO:0008569] (molecular function) Relationships: is a type of GO:0003777 References: PMID:15659646, PMID:32842864 Sources: GOC:mah, GOC:vw Also known as: ATP-dependent microtubule motor activity, minus-end-directed, ATP-dependent minus-end-directed microtubule motor activity, microtubule motor activity, minus-end-directed, minus-end-directed ATP-dependent microtubule motor activity, dynein ATPase, kinesin ATP phosphohydrolase (minus-end-directed), minus-end-directed kinesin ATPase activity Definition: A motor activity that generates movement along a microtubule toward the minus end, driven by ATP hydrolysis.